interleukin-26 binding [GO:0045512] (molecular function) Relationships: is_a cytokine binding [GO:0019955] Sources: GOC:go_curators Definition: Binding to interleukin-26. Also known as: IL-26 binding